regulation of fatty acid metabolic process [GO:0019217] (BP) Definition: Any process that modulates the frequency, rate or extent of the chemical reactions and pathways involving fatty acids. Relationships: is a type of regulation of ketone metabolic process [GO:0010565]; is a type of regulation of lipid metabolic process [GO:0019216]; is a type of GO:0062012; regulates fatty acid metabolic process [GO:0006631] Sources: GOC:go_curators Also known as: regulation of fatty acid metabolism Subtypes: GO:0042304, GO:0045922, positive regulation of fatty acid metabolic process [GO:0045923], regulation of fatty acid oxidation [GO:0046320], regulation of acyl-CoA biosynthetic process [GO:0050812], regulation of jasmonic acid metabolic process [GO:0080140], regulation of palmitic acid catabolic process [GO:0106393], regulation of methane biosynthetic process from 3-(methylthio)propionic acid [GO:1900333], regulation of butyryl-CoA catabolic process to butanol [GO:1900497]